{
  "gene_symbol": "CILK1",
  "term_id": "GO:0005929",
  "gene": "UniProtKB:Q9UPZ9",
  "gene_name": "Serine_threonine-protein kinase ICK",
  "term_label": "cilium"
}